{
  "gene": "UniProtKB:Q9BXK1",
  "gene_symbol": "KLF16",
  "term_id": "GO:0005634",
  "gene_name": "Krueppel-like factor 16",
  "term_label": "nucleus"
}